positive regulation of establishment of T cell polarity [GO:1903905] (biological process) References: PMID:23575248 Sources: GOC:TermGenie, GOC:als, GO_REF:0000058 Definition: Any process that activates or increases the frequency, rate or extent of establishment of T cell polarity. Also known as: positive regulation of T cell polarization, positive regulation of T lymphocyte polarization, positive regulation of T-cell polarization, positive regulation of establishment of T lymphocyte polarity, positive regulation of establishment of T-cell polarity, positive regulation of establishment of T-lymphocyte polarity, up regulation of T cell polarization, up regulation of T lymphocyte polarization, up regulation of T-cell polarization, up regulation of establishment of T cell polarity, up regulation of establishment of T lymphocyte polarity, up regulation of establishment of T-cell polarity, up regulation of establishment of T-lymphocyte polarity, up-regulation of T cell polarization, up-regulation of T lymphocyte polarization, up-regulation of T-cell polarization, up-regulation of establishment of T cell polarity, up-regulation of establishment of T lymphocyte polarity, up-regulation of establishment of T-cell polarity, up-regulation of establishment of T-lymphocyte polarity, upregulation of T cell polarization, upregulation of T lymphocyte polarization, upregulation of T-cell polarization, upregulation of establishment of T cell polarity, upregulation of establishment of T lymphocyte polarity, upregulation of establishment of T-cell polarity, upregulation of establishment of T-lymphocyte polarity, activation of T cell polarization, activation of T lymphocyte polarization, activation of T-cell polarization, activation of establishment of T cell polarity, activation of establishment of T lymphocyte polarity, activation of establishment of T-cell polarity, activation of establishment of T-lymphocyte polarity Relationships: is a type of positive regulation of T cell activation [GO:0050870]; is a type of GO:1903903; RO_0002213 establishment of T cell polarity [GO:0001768]